{
  "gene_name": "Twinfilin-1",
  "term_id": "GO:0010591",
  "term_label": "regulation of lamellipodium assembly",
  "gene": "UniProtKB:Q12792",
  "gene_symbol": "TWF1"
}